{
  "gene_symbol": "ZNF723",
  "gene_name": "Zinc finger protein 723",
  "term_label": "regulation of DNA-templated transcription",
  "gene": "UniProtKB:P0DPD5",
  "term_id": "GO:0006355"
}